neuron projection terminus [GO:0044306] (cellular component) Sources: GOC:jl Subtypes: axon terminus [GO:0043679] Definition: The specialized, terminal region of a neuron projection such as an axon or a dendrite. Also known as: neuron projection terminal, neuron terminal specialization, nerve terminal Relationships: is a type of GO:0110165; is part of neuron projection [GO:0043005]